{
  "gene_symbol": "CUL4A",
  "term_id": "GO:0031464",
  "gene_name": "Cullin-4A",
  "term_label": "Cul4A-RING E3 ubiquitin ligase complex",
  "gene": "UniProtKB:Q13619"
}